negative regulation of leukocyte cell-cell adhesion [GO:1903038] (biological process) Note: Exogenous expression of ASS1 or NOS3 in HUVECs enhances NO production and inhibits monocyte adhesion Also known as: down regulation of leukocyte adhesion, down regulation of leukocyte cell adhesion, down regulation of leukocyte cell-cell adhesion, down-regulation of leukocyte adhesion, down-regulation of leukocyte cell adhesion, down-regulation of leukocyte cell-cell adhesion, downregulation of leukocyte adhesion, downregulation of leukocyte cell adhesion, downregulation of leukocyte cell-cell adhesion, negative regulation of leukocyte adhesion, negative regulation of leukocyte cell adhesion, inhibition of leukocyte adhesion, inhibition of leukocyte cell adhesion, inhibition of leukocyte cell-cell adhesion Definition: Any process that stops, prevents or reduces the frequency, rate or extent of leukocyte cell-cell adhesion. References: PMID:21106532 Sources: GOC:BHF, GOC:TermGenie, GOC:rl, GO_REF:0000058 Relationships: is a type of negative regulation of cell-cell adhesion [GO:0022408]; is a type of regulation of leukocyte cell-cell adhesion [GO:1903037]; negatively regulates leukocyte cell-cell adhesion [GO:0007159] Subtypes: GO:0050868, negative regulation of monocyte aggregation [GO:1900624], negative regulation of leukocyte adhesion to vascular endothelial cell [GO:1904995], negative regulation of thymocyte aggregation [GO:2000399], GO:2000429